positive regulation of peptidyl-tyrosine autophosphorylation [GO:1900086] (biological process) Definition: Any process that activates or increases the frequency, rate or extent of peptidyl-tyrosine autophosphorylation. Sources: GOC:TermGenie, GOC:bf Also known as: positive regulation of tyrosine autophosphorylation, up regulation of peptidyl-tyrosine autophosphorylation, up regulation of tyrosine autophosphorylation, up-regulation of peptidyl-tyrosine autophosphorylation, up-regulation of tyrosine autophosphorylation, upregulation of peptidyl-tyrosine autophosphorylation, upregulation of tyrosine autophosphorylation, activation of peptidyl-tyrosine autophosphorylation, activation of receptor tyrosine kinase autophosphorylation, activation of tyrosine autophosphorylation, positive regulation of receptor tyrosine kinase autophosphorylation, up regulation of receptor tyrosine kinase autophosphorylation, up-regulation of receptor tyrosine kinase autophosphorylation, upregulation of receptor tyrosine kinase autophosphorylation Relationships: is a type of GO:0031954; is a type of positive regulation of peptidyl-tyrosine phosphorylation [GO:0050731]; is a type of regulation of peptidyl-tyrosine autophosphorylation [GO:1900084]; positively regulates GO:0038083